{
  "gene_symbol": "VMO1",
  "term_id": "GO:0005615",
  "gene_name": "Vitelline membrane outer layer protein 1 homolog",
  "term_label": "extracellular space",
  "gene": "UniProtKB:Q7Z5L0"
}